{
  "gene_symbol": "PDHX",
  "gene_name": "Pyruvate dehydrogenase protein X component, mitochondrial",
  "term_label": "Unknown molecular function",
  "gene": "UniProtKB:O00330",
  "term_id": "UNKNOWN:0001"
}